{
  "gene_name": "Putative E3 ubiquitin-protein ligase makorin-4",
  "term_label": "protein ubiquitination",
  "term_id": "GO:0016567",
  "gene": "UniProtKB:Q13434",
  "gene_symbol": "MKRN4P"
}